{
  "gene_name": "ADP-ribosylation factor-like protein 2",
  "term_id": "GO:0005525",
  "gene": "UniProtKB:P36404",
  "term_label": "GTP binding",
  "gene_symbol": "ARL2"
}